deoxysarpagine hydroxylase activity [GO:0033775] (MF) Sources: EC:1.14.14.136, RHEA:14237 Also known as: 10-deoxysarpagine,NADPH:oxygen oxidoreductase (10-hydroxylating) activity, DOSH Relationships: is a type of oxidoreductase activity, acting on paired donors, with incorporation or reduction of molecular oxygen, NAD(P)H as one donor, and incorporation of one atom of oxygen [GO:0016709] Definition: Catalysis of the reaction: 10-deoxysarpagine + H+ + NADPH + O2 = H2O + NADP+ + sarpagine.